{
  "term_id": "GO:0005634",
  "gene": "UniProtKB:O00425",
  "gene_name": "Insulin-like growth factor 2 mRNA-binding protein 3",
  "term_label": "nucleus",
  "gene_symbol": "IGF2BP3"
}